{
  "term_label": "mitochondrion",
  "gene": "UniProtKB:Q7Z6M4",
  "term_id": "GO:0005739",
  "gene_symbol": "MTERF4",
  "gene_name": "Transcription termination factor 4, mitochondrial"
}